{
  "gene": "UniProtKB:Q9UM63",
  "term_id": "GO:0001228",
  "gene_name": "Zinc finger protein PLAGL1",
  "term_label": "DNA-binding transcription activator activity, RNA polymerase II-specific",
  "gene_symbol": "PLAGL1"
}